gamma-aminobutyric acid transport [GO:0015812] (biological process) Sources: GOC:go_curators, ISBN:0198506732 Relationships: is_a amino acid transport [GO:0006865]; is_a carboxylic acid transport [GO:0046942]; is a type of nitrogen compound transport [GO:0071705] Definition: The directed movement of gamma-aminobutyric acid (GABA, 4-aminobutyrate), an amino acid which acts as a neurotransmitter in some organisms, into, out of or within a cell, or between cells, by means of some agent such as a transporter or pore. Note: See also the biological process term 'neurotransmitter transport ; GO:0006836'. Also known as: 4-aminobutanoate transport, 4-aminobutyrate transport, GABA transport Subtypes: gamma-aminobutyric acid secretion [GO:0014051], gamma-aminobutyric acid reuptake [GO:0051936], gamma-aminobutyric acid import [GO:0051939]